{
  "gene": "UniProtKB:Q08209",
  "term_id": "GO:0033173",
  "gene_name": "Protein phosphatase 3 catalytic subunit alpha",
  "term_label": "calcineurin-NFAT signaling cascade",
  "gene_symbol": "PPP3CA"
}